{
  "gene_name": "Prefoldin subunit 2",
  "gene_symbol": "PFDN2",
  "term_label": "protein folding chaperone",
  "gene": "UniProtKB:Q9UHV9",
  "term_id": "GO:0044183"
}